{
  "gene": "UniProtKB:P28290",
  "gene_name": "Protein ITPRID2",
  "gene_symbol": "ITPRID2",
  "term_label": "Unknown biological process",
  "term_id": "UNKNOWN:0002"
}